{
  "term_label": "actin filament",
  "gene": "UniProtKB:P0CG38",
  "gene_symbol": "POTEI",
  "gene_name": "POTE ankyrin domain family member I",
  "term_id": "GO:0005884"
}